3-deoxy-manno-octulosonate-8-phosphatase activity [GO:0019143] (molecular function) Definition: Catalysis of the reaction: 8-phospho-3-deoxy-D-manno-oct-2-ulosonate + H2O = 3-deoxy-D-manno-octulosonate + phosphate. Sources: EC:3.1.3.45, RHEA:11500 Also known as: 3-deoxy-D-manno-octulosonate-8-phosphate 8-phosphohydrolase activity Relationships: is a type of phosphatase activity [GO:0016791]